{
  "gene_name": "DnaJ homolog subfamily C member 7",
  "term_id": "UNKNOWN:0003",
  "gene_symbol": "DNAJC7",
  "term_label": "Unknown cellular component",
  "gene": "UniProtKB:Q99615"
}